{
  "term_label": "preribosome, small subunit precursor",
  "gene_symbol": "RIOK1",
  "gene_name": "Serine_threonine-protein kinase RIO1",
  "gene": "UniProtKB:Q9BRS2",
  "term_id": "GO:0030688"
}